{
  "gene": "UniProtKB:Q9BRT8",
  "gene_symbol": "ZNG1A",
  "term_label": "zinc chaperone activity",
  "term_id": "GO:0140827",
  "gene_name": "Zinc-regulated GTPase metalloprotein activator 1A"
}